{
  "gene_name": "Dickkopf-like protein 1",
  "term_label": "co-receptor binding",
  "gene": "UniProtKB:Q9UK85",
  "gene_symbol": "DKKL1",
  "term_id": "GO:0039706"
}